{
  "gene_symbol": "SLC4A3",
  "gene": "UniProtKB:P48751",
  "term_id": "GO:0015701",
  "gene_name": "Anion exchange protein 3",
  "term_label": "bicarbonate transport"
}